{
  "gene": "UniProtKB:Q6NT32",
  "gene_symbol": "CES5A",
  "gene_name": "Carboxylesterase 5A",
  "term_label": "carboxylesterase activity",
  "term_id": "GO:0106435"
}